{
  "gene": "UniProtKB:Q8NGZ4",
  "term_id": "GO:0004984",
  "term_label": "olfactory receptor activity",
  "gene_name": "Olfactory receptor 2G3",
  "gene_symbol": "OR2G3"
}